{
  "gene": "UniProtKB:Q9H999",
  "gene_name": "Pantothenate kinase 3",
  "gene_symbol": "PANK3",
  "term_id": "GO:0005829",
  "term_label": "cytosol"
}